N,N'-diacetylchitobiose import [GO:1902815] (biological process) Relationships: is a type of carbohydrate derivative transport [GO:1901264] Definition: The directed movement of N,N'-diacetylchitobiose into a cell or organelle. References: PMID:9405618 Sources: GOC:TermGenie, GOC:am, GO_REF:0000073